excitatory synapse pruning [GO:1905805] (biological process) References: PMID:27779093 Sources: GOC:TermGenie, GO_REF:0000079 Definition: The disaggregation of an excitatory synapse into its constituent components. Regulation: regulated by regulation of excitatory synapse pruning [GO:1905810]; negatively regulated by negative regulation of excitatory synapse pruning [GO:1905811] Relationships: is_a GO:0098883 Also known as: synapse clearance, synapse disassembly, synapse elimination, synapse removal